sphinganine-1-phosphate metabolic process [GO:0006668] (BP) Relationships: is a type of phospholipid metabolic process [GO:0006644]; is a type of GO:0006665 Also known as: dihydrosphingosine-1-phosphate metabolic process, dihydrosphingosine-1-phosphate metabolism, sphinganine-1-phosphate metabolism Subtypes: sphinganine-1-phosphate biosynthetic process [GO:0006669], sphinganine-1-phosphate catabolic process [GO:0051874] Definition: The chemical reactions and pathways involving sphinganine-1-phosphate, the phosphorylated derivative of D-erythro-2-amino-1,3-octadecanediol. Sources: GOC:ai